establishment or maintenance of cell type involved in phenotypic switching [GO:0044663] (biological process) Relationships: is a type of cellular process [GO:0009987]; is part of GO:0036166 Definition: A cellular process of the specification, formation or maintenance of an alternative cell type, occurring as part of the process of phenotypic switching. Phenotypic switching begins with changes in cell morphology and altered gene expression patterns and ends when the morphology of a population of cells has reverted back to the default state, accompanied by altered expression patterns. Sources: GOC:jl